{
  "gene_symbol": "IFNB1",
  "term_label": "natural killer cell activation involved in immune response",
  "gene": "UniProtKB:P01574",
  "gene_name": "Interferon beta",
  "term_id": "GO:0002323"
}